{
  "gene_name": "Ras-related protein Rab-40C",
  "gene_symbol": "RAB40C",
  "term_id": "GO:0008021",
  "gene": "UniProtKB:Q96S21",
  "term_label": "synaptic vesicle"
}